{
  "gene": "UniProtKB:Q16348",
  "gene_symbol": "SLC15A2",
  "gene_name": "Solute carrier family 15 member 2",
  "term_label": "plasma membrane",
  "term_id": "GO:0005886"
}